{
  "term_label": "Unknown molecular function",
  "gene": "UniProtKB:Q5T686",
  "term_id": "UNKNOWN:0001",
  "gene_name": "Arginine vasopressin-induced protein 1",
  "gene_symbol": "AVPI1"
}